{
  "gene_symbol": "MYO6",
  "term_id": "GO:0051015",
  "gene": "UniProtKB:Q9UM54",
  "gene_name": "Unconventional myosin-VI",
  "term_label": "actin filament binding"
}